{
  "gene_symbol": "BLM",
  "gene_name": "RecQ-like DNA helicase BLM",
  "gene": "UniProtKB:P54132",
  "term_label": "double-strand break repair via homologous recombination",
  "term_id": "GO:0000724"
}